{
  "term_id": "GO:0033883",
  "gene_name": "Chronophin",
  "term_label": "pyridoxal phosphatase activity",
  "gene": "UniProtKB:Q96GD0",
  "gene_symbol": "PDXP"
}